{
  "gene_name": "Putative uncharacterized protein encoded by LINC01545",
  "gene_symbol": "LINC01545",
  "term_label": "Unknown molecular function",
  "gene": "UniProtKB:Q5VT33",
  "term_id": "UNKNOWN:0001"
}